{
  "gene_symbol": "EID2B",
  "gene_name": "EP300-interacting inhibitor of differentiation 2B",
  "term_id": "GO:0003714",
  "gene": "UniProtKB:Q96D98",
  "term_label": "transcription corepressor activity"
}